{
  "term_label": "DNA replication factor A complex",
  "gene_symbol": "RPA2",
  "gene_name": "Replication protein A 32 kDa subunit",
  "term_id": "GO:0005662",
  "gene": "UniProtKB:P15927"
}